{
  "gene_symbol": "NVL",
  "term_id": "GO:0016887",
  "gene": "UniProtKB:O15381",
  "gene_name": "Nuclear valosin-containing protein-like",
  "term_label": "ATP hydrolysis activity"
}